dUDP biosynthetic process [GO:0006227] (biological process) Also known as: dUDP anabolism, dUDP biosynthesis, dUDP formation, dUDP synthesis Definition: The chemical reactions and pathways resulting in the formation of dUDP, deoxyuridine diphosphate (2'-deoxy-5'-uridylyl phosphate). Relationships: is a type of pyrimidine deoxyribonucleoside diphosphate biosynthetic process [GO:0009197]; is a type of pyrimidine deoxyribonucleotide biosynthetic process [GO:0009221]; is a type of dUDP metabolic process [GO:0046077] Sources: ISBN:0198506732